{
  "term_id": "GO:0030335",
  "gene_name": "C-C motif chemokine 13",
  "gene_symbol": "CCL13",
  "term_label": "positive regulation of cell migration",
  "gene": "UniProtKB:Q99616"
}